{
  "term_id": "GO:0002223",
  "gene_name": "NKG2-C type II integral membrane protein",
  "gene_symbol": "KLRC2",
  "gene": "UniProtKB:P26717",
  "term_label": "stimulatory C-type lectin receptor signaling pathway"
}